{
  "term_label": "GPI anchor biosynthetic process",
  "gene_symbol": "PIGM",
  "term_id": "GO:0006506",
  "gene": "UniProtKB:Q9H3S5",
  "gene_name": "GPI mannosyltransferase 1"
}